{
  "term_id": "UNKNOWN:0001",
  "gene_symbol": "ATXN10",
  "gene": "UniProtKB:Q9UBB4",
  "term_label": "Unknown molecular function",
  "gene_name": "Ataxin-10"
}